{
  "gene_name": "Phosphatidylinositol 4-phosphate 5-kinase type-1 alpha",
  "gene": "UniProtKB:Q99755",
  "gene_symbol": "PIP5K1A",
  "term_label": "phosphatidylinositol phosphate biosynthetic process",
  "term_id": "GO:0046854"
}